{
  "term_id": "GO:0006357",
  "gene_name": "Zinc finger and SCAN domain-containing protein 22",
  "term_label": "regulation of transcription by RNA polymerase II",
  "gene": "UniProtKB:P10073",
  "gene_symbol": "ZSCAN22"
}